{
  "term_id": "GO:0006868",
  "gene_symbol": "SLC38A3",
  "gene_name": "Sodium-coupled neutral amino acid transporter 3",
  "gene": "UniProtKB:Q99624",
  "term_label": "glutamine transport"
}